{
  "gene": "UniProtKB:Q13153",
  "term_label": "cellular response to starvation",
  "term_id": "GO:0009267",
  "gene_name": "Serine_threonine-protein kinase PAK 1",
  "gene_symbol": "PAK1"
}